{
  "term_id": "GO:0097632",
  "gene_name": "Beclin 1-associated autophagy-related key regulator",
  "gene": "UniProtKB:Q6ZNE5",
  "term_label": "extrinsic component of phagophore assembly site membrane",
  "gene_symbol": "ATG14"
}